{
  "gene_symbol": "AADACL4",
  "term_id": "UNKNOWN:0003",
  "gene_name": "Arylacetamide deacetylase-like 4",
  "term_label": "Unknown cellular component",
  "gene": "UniProtKB:Q5VUY2"
}